{
  "gene_name": "TRAF-type zinc finger domain-containing protein 1",
  "term_id": "GO:0045824",
  "gene_symbol": "TRAFD1",
  "gene": "UniProtKB:O14545",
  "term_label": "negative regulation of innate immune response"
}